alpha-D-xyloside xylohydrolase [GO:0061634] (molecular function) Relationships: is a type of GO:0004553 Also known as: alpha-xylosidase Definition: Catalysis of the hydrolysis of terminal, non-reducing alpha-D-xylose residues with release of alpha-D-xylose. Sources: EC:3.2.1.177